{
  "gene_symbol": "NACC2",
  "gene": "UniProtKB:Q96BF6",
  "gene_name": "Nucleus accumbens-associated protein 2",
  "term_label": "RNA polymerase II cis-regulatory region sequence-specific DNA binding",
  "term_id": "GO:0000978"
}